{
  "gene": "UniProtKB:Q8WU68",
  "term_label": "U2AF complex",
  "gene_name": "Splicing factor U2AF 26 kDa subunit",
  "gene_symbol": "U2AF1L4",
  "term_id": "GO:0089701"
}